cholesterol biosynthetic process [GO:0006695] (BP) Definition: The chemical reactions and pathways resulting in the formation of cholesterol, cholest-5-en-3 beta-ol, the principal sterol of vertebrates and the precursor of many steroids, including bile acids and steroid hormones. Relationships: is a type of GO:0008203; is a type of sterol biosynthetic process [GO:0016126]; is a type of secondary alcohol biosynthetic process [GO:1902653] Also known as: cholesterol anabolism, cholesterol biosynthesis, cholesterol formation, cholesterol synthesis Sources: GOC:ai Subtypes: GO:0033488, cholesterol biosynthetic process via desmosterol [GO:0033489], cholesterol biosynthetic process via lathosterol [GO:0033490] Regulation: regulated by regulation of cholesterol biosynthetic process [GO:0045540]; negatively regulated by negative regulation of cholesterol biosynthetic process [GO:0045541]; positively regulated by positive regulation of cholesterol biosynthetic process [GO:0045542]